{
  "term_id": "GO:0030018",
  "gene": "UniProtKB:Q86VF7",
  "term_label": "Z disc",
  "gene_name": "Nebulin-related-anchoring protein",
  "gene_symbol": "NRAP"
}